{
  "gene_name": "G-protein coupled receptor-associated sorting protein 2",
  "term_label": "Unknown biological process",
  "gene_symbol": "GPRASP2",
  "gene": "UniProtKB:Q96D09",
  "term_id": "UNKNOWN:0002"
}